{
  "term_id": "GO:0004714",
  "gene_name": "High affinity nerve growth factor receptor",
  "gene_symbol": "NTRK1",
  "term_label": "transmembrane receptor protein tyrosine kinase activity",
  "gene": "UniProtKB:P04629"
}